{
  "term_id": "GO:0022625",
  "gene_symbol": "RPL24",
  "gene_name": "Large ribosomal subunit protein eL24",
  "gene": "UniProtKB:P83731",
  "term_label": "cytosolic large ribosomal subunit"
}